regulation of extracellular matrix disassembly [GO:0010715] (biological process) Sources: GOC:BHF, GOC:dph, GOC:tb Relationships: is a type of GO:1903053; regulates extracellular matrix disassembly [GO:0022617] Also known as: regulation of extracellular matrix breakdown, regulation of extracellular matrix degradation Definition: Any process that modulates the rate, frequency or extent of extracellular matrix disassembly. Extracellular matrix disassembly is a process that results in the breakdown of the extracellular matrix. Subtypes: negative regulation of extracellular matrix disassembly [GO:0010716], positive regulation of extracellular matrix disassembly [GO:0090091]